{
  "term_id": "GO:0016020",
  "gene_name": "Magnesium transporter NIPA3",
  "term_label": "membrane",
  "gene_symbol": "NIPAL1",
  "gene": "UniProtKB:Q6NVV3"
}